{
  "gene_name": "Large ribosomal subunit protein uL1m",
  "gene": "UniProtKB:Q9BYD6",
  "gene_symbol": "MRPL1",
  "term_id": "GO:0003729",
  "term_label": "mRNA binding"
}